{
  "gene_name": "C-type lectin domain family 2 member B",
  "gene": "UniProtKB:Q92478",
  "gene_symbol": "CLEC2B",
  "term_id": "GO:0046703",
  "term_label": "natural killer cell lectin-like receptor binding"
}